{
  "gene_symbol": "SLC4A9",
  "term_id": "GO:0005886",
  "gene": "UniProtKB:Q96Q91",
  "term_label": "plasma membrane",
  "gene_name": "Anion exchange protein 4"
}